{
  "gene_symbol": "NUDT5",
  "gene": "UniProtKB:Q9UKK9",
  "gene_name": "ADP-sugar pyrophosphatase",
  "term_label": "nucleoside phosphate metabolic process",
  "term_id": "GO:0006753"
}